{
  "term_label": "Unknown biological process",
  "gene_name": "Transmembrane protein 91",
  "term_id": "UNKNOWN:0002",
  "gene_symbol": "TMEM91",
  "gene": "UniProtKB:Q6ZNR0"
}